{
  "term_label": "neuron differentiation",
  "term_id": "GO:0030182",
  "gene_name": "Tubulin alpha-1C chain",
  "gene_symbol": "TUBA1C",
  "gene": "UniProtKB:Q9BQE3"
}